meiotic chromosome separation [GO:0051307] (biological process) Definition: The process in which chromosomes are physically detached from each other during meiosis. Sources: GOC:ai Also known as: chromosome separation during meiosis, meiotic chromosome resolution Relationships: is a type of chromosome separation [GO:0051304]; is a type of meiotic cell cycle process [GO:1903046]; is part of meiotic chromosome segregation [GO:0045132] Subtypes: male meiosis chromosome separation [GO:0051308], female meiosis chromosome separation [GO:0051309], meiotic sister chromatid separation [GO:0051757] Regulation: regulated by regulation of meiotic chromosome separation [GO:1905132]; negatively regulated by GO:1905133; positively regulated by positive regulation of meiotic chromosome separation [GO:1905134]